guaiacyl lignin catabolic process [GO:1901062] (biological process) Also known as: G-lignin catabolic process, guaiacyl lignin breakdown, guaiacyl lignin catabolism, guaiacyl lignin degradation Definition: The chemical reactions and pathways resulting in the breakdown of guaiacyl lignin. Relationships: is a type of lignin catabolic process [GO:0046274] Sources: GOC:TermGenie, GOC:mengo_curators